TIRAP-dependent toll-like receptor 4 signaling pathway [GO:0035665] (biological process) Definition: The series of molecular signals initiated by a ligand binding to a toll-like receptor 4 where the TIRAP/MAL adaptor mediates transduction of the signal. Toll-like 4 receptors are pattern recognition receptors that bind bacterial lipopolysaccharide (LPS) to initiate an innate immune response. References: PMID:12447441 Sources: GOC:BHF Also known as: MAL-dependent toll-like receptor 4 signaling pathway, MyD88 adapter-like dependent toll-like receptor 4 signaling pathway, TIRAP-dependent TLR4 signaling pathway, TIRAP-dependent toll-like receptor 4 signalling pathway Relationships: is a type of toll-like receptor 4 signaling pathway [GO:0034142]; is a type of TIRAP-dependent toll-like receptor signaling pathway [GO:0035664]